regulation of smooth muscle hypertrophy [GO:1905147] (BP) Subtypes: negative regulation of smooth muscle hypertrophy [GO:1905148], positive regulation of smooth muscle hypertrophy [GO:1905149] References: PMID:22161164 Sources: GOC:BHF, GOC:BHF_miRNA, GOC:TermGenie, GOC:bc, GO_REF:0000058 Definition: Any process that modulates the frequency, rate or extent of smooth muscle hypertrophy. Relationships: is a type of regulation of muscle hypertrophy [GO:0014743]; is a type of regulation of muscle adaptation [GO:0043502]; regulates GO:0014895